{
  "gene": "UniProtKB:Q9Y6R9",
  "gene_name": "Centrosomal protein CCDC61",
  "term_id": "UNKNOWN:0001",
  "gene_symbol": "CCDC61",
  "term_label": "Unknown molecular function"
}